{
  "term_id": "GO:0005509",
  "gene_symbol": "AOAH",
  "gene": "UniProtKB:P28039",
  "gene_name": "Acyloxyacyl hydrolase",
  "term_label": "calcium ion binding"
}